{
  "gene_name": "Sodium- and chloride-dependent GABA transporter 3",
  "gene": "UniProtKB:P48066",
  "term_id": "GO:0005332",
  "gene_symbol": "SLC6A11",
  "term_label": "gamma-aminobutyric acid:sodium:chloride symporter activity"
}